{
  "gene_symbol": "GCN1",
  "gene_name": "Stalled ribosome sensor GCN1",
  "term_label": "protein kinase regulator activity",
  "term_id": "GO:0019887",
  "gene": "UniProtKB:Q92616"
}